{
  "term_id": "GO:0007399",
  "gene": "UniProtKB:Q9BWV1",
  "term_label": "nervous system development",
  "gene_name": "Brother of CDO",
  "gene_symbol": "BOC"
}